{
  "gene": "UniProtKB:P01700",
  "term_id": "GO:0019814",
  "gene_symbol": "IGLV1-47",
  "term_label": "immunoglobulin complex",
  "gene_name": "Immunoglobulin lambda variable 1-47"
}